{
  "gene_symbol": "TUSC2",
  "gene_name": "Tumor suppressor candidate 2",
  "term_id": "GO:0005739",
  "gene": "UniProtKB:O75896",
  "term_label": "mitochondrion"
}